{
  "gene_name": "Protein furry homolog",
  "term_id": "GO:0030427",
  "term_label": "site of polarized growth",
  "gene_symbol": "FRY",
  "gene": "UniProtKB:Q5TBA9"
}